{
  "term_label": "Unknown cellular component",
  "gene_name": "5'-nucleotidase domain-containing protein 2",
  "term_id": "UNKNOWN:0003",
  "gene": "UniProtKB:Q9H857",
  "gene_symbol": "NT5DC2"
}